{
  "gene_symbol": "CAPN3",
  "term_id": "GO:0004198",
  "gene_name": "Calpain-3",
  "term_label": "calcium-dependent cysteine-type endopeptidase activity",
  "gene": "UniProtKB:P20807"
}